cellular response to nutrient levels [GO:0031669] (biological process) Sources: GOC:mah Subtypes: cellular response to starvation [GO:0009267], negative regulation of ribosomal protein gene transcription from RNA polymerase II promoter in response to nutrient levels [GO:0010691], cellular response to nutrient [GO:0031670], cellular response to nitrogen levels [GO:0043562], GO:0080029, cellular response to oxygen-glucose deprivation [GO:0090650] Definition: Any process that results in a change in state or activity of a cell (in terms of movement, secretion, enzyme production, gene expression, etc.) as a result of a stimulus reflecting the presence, absence, or concentration of nutrients. Relationships: is a type of response to nutrient levels [GO:0031667]; is a type of cellular response to stimulus [GO:0051716]